(S)-citramalyl-CoA lyase activity [GO:0047777] (molecular function) Sources: EC:4.1.3.25, RHEA:22612 Definition: Catalysis of the reaction: (3S)-citramalyl-CoA = acetyl-CoA + pyruvate. Relationships: is a type of oxo-acid-lyase activity [GO:0016833] Also known as: citramalyl-CoA lyase activity, (+)-CMA-CoA lyase activity, (3S)-citramalyl-CoA lyase activity, (3S)-citramalyl-CoA pyruvate-lyase (acetyl-CoA-forming), (3S)-citramalyl-CoA pyruvate-lyase activity, citramalyl coenzyme A lyase activity